{
  "gene": "UniProtKB:Q9Y689",
  "gene_symbol": "ARL5A",
  "term_id": "GO:0005802",
  "term_label": "trans-Golgi network",
  "gene_name": "ADP-ribosylation factor-like protein 5A"
}